{
  "gene": "UniProtKB:Q99788",
  "gene_symbol": "CMKLR1",
  "gene_name": "Chemerin-like receptor 1",
  "term_label": "regulation of calcium-mediated signaling",
  "term_id": "GO:0050848"
}